{
  "term_label": "nucleus",
  "gene_name": "Tubulin gamma-1 chain",
  "gene_symbol": "TUBG1",
  "term_id": "GO:0005634",
  "gene": "UniProtKB:P23258"
}